positive regulation of substrate adhesion-dependent cell spreading [GO:1900026] (biological process) Definition: Any process that activates or increases the frequency, rate or extent of substrate adhesion-dependent cell spreading. Relationships: is a type of positive regulation of cell-substrate adhesion [GO:0010811]; is a type of regulation of substrate adhesion-dependent cell spreading [GO:1900024]; RO_0002213 substrate adhesion-dependent cell spreading [GO:0034446] Sources: GOC:TermGenie, GOC:yaf Also known as: positive regulation of cell spreading during cell substrate adhesion, positive regulation of substrate adhesion dependent cell spreading, up regulation of cell spreading during cell substrate adhesion, up regulation of substrate adhesion dependent cell spreading, up regulation of substrate adhesion-dependent cell spreading